{
  "gene": "UniProtKB:Q8IW92",
  "term_id": "GO:0005773",
  "gene_symbol": "GLB1L2",
  "gene_name": "Beta-galactosidase-1-like protein 2",
  "term_label": "vacuole"
}